NADH dehydrogenase (quinone) (non-electrogenic) activity [GO:0050136] (molecular function) Also known as: NADH:ubiquinone reductase (non-electrogenic) activity, NADH dehydrogenase (quinone) activity Sources: RHEA:46160 Relationships: is a type of GO:0003954; is a type of NAD(P)H dehydrogenase (quinone) activity [GO:0003955] Definition: Catalysis of the reaction: NADH + H+ + a quinone = NAD+ + a quinol. Subtypes: NADH dehydrogenase (menaquinone) (non-electrogenic) activity [GO:0103036], NADH dehydrogenase (ubiquinone) (non-electrogenic) activity [GO:0120555]